{
  "gene_name": "Phosphoenolpyruvate carboxykinase [GTP], mitochondrial",
  "gene_symbol": "PCK2",
  "term_id": "GO:0006107",
  "term_label": "oxaloacetate metabolic process",
  "gene": "UniProtKB:Q16822"
}